{
  "gene_name": "Gamma-aminobutyric acid receptor subunit alpha-6",
  "term_id": "GO:1902476",
  "gene": "UniProtKB:Q16445",
  "gene_symbol": "GABRA6",
  "term_label": "chloride transmembrane transport"
}